{
  "term_id": "GO:0009897",
  "gene_symbol": "GFRAL",
  "gene": "UniProtKB:Q6UXV0",
  "gene_name": "GDNF family receptor alpha-like",
  "term_label": "external side of plasma membrane"
}